{
  "gene_symbol": "PTGER3",
  "term_label": "negative regulation of gastric acid secretion",
  "gene_name": "Prostaglandin E2 receptor EP3 subtype",
  "gene": "UniProtKB:P43115",
  "term_id": "GO:0060455"
}